type IV site-specific deoxyribonuclease complex [GO:0032068] (cellular component) Definition: A complex consisting of two proteins which acts as an endonuclease in DNA sequences containing a specific modified recognition site. Modifications may include methylation, hydroxymethylation, and glucosyl-hydroxymethylation. References: PMID:12654995 Also known as: type IV restriction enzyme complex Relationships: is a type of GO:1905347; is part of cytoplasm [GO:0005737]